{
  "term_label": "transcription corepressor activity",
  "gene_symbol": "RCOR3",
  "term_id": "GO:0003714",
  "gene": "UniProtKB:Q9P2K3",
  "gene_name": "REST corepressor 3"
}